{
  "term_id": "UNKNOWN:0002",
  "term_label": "Unknown biological process",
  "gene_name": "Solute carrier family 22 member 23",
  "gene": "UniProtKB:A1A5C7",
  "gene_symbol": "SLC22A23"
}